regulation of progesterone biosynthetic process [GO:2000182] (biological process) Definition: Any process that modulates the frequency, rate or extent of progesterone biosynthetic process. Also known as: regulation of progesterone anabolism, regulation of progesterone biosynthesis, regulation of progesterone formation, regulation of progesterone synthesis Relationships: is a type of regulation of ketone biosynthetic process [GO:0010566]; is a type of regulation of hormone biosynthetic process [GO:0046885]; is a type of regulation of steroid biosynthetic process [GO:0050810]; regulates progesterone biosynthetic process [GO:0006701] Sources: GOC:dph Subtypes: negative regulation of progesterone biosynthetic process [GO:2000183], positive regulation of progesterone biosynthetic process [GO:2000184]